{
  "gene_symbol": "MAP2K1",
  "term_id": "GO:0000165",
  "gene": "UniProtKB:Q02750",
  "gene_name": "Dual specificity mitogen-activated protein kinase kinase 1",
  "term_label": "MAPK cascade"
}